{
  "gene_name": "Neurobeachin-like protein 1",
  "term_label": "Unknown molecular function",
  "gene_symbol": "NBEAL1",
  "term_id": "UNKNOWN:0001",
  "gene": "UniProtKB:Q6ZS30"
}